{
  "gene": "UniProtKB:A8TX70",
  "term_id": "UNKNOWN:0001",
  "term_label": "Unknown molecular function",
  "gene_symbol": "COL6A5",
  "gene_name": "Collagen alpha-5(VI) chain"
}